{
  "gene": "UniProtKB:Q6ZRR5",
  "gene_name": "TLC domain-containing protein 5",
  "gene_symbol": "TLCD5",
  "term_id": "UNKNOWN:0003",
  "term_label": "Unknown cellular component"
}